{
  "term_id": "GO:0005929",
  "term_label": "cilium",
  "gene": "UniProtKB:P56597",
  "gene_name": "Nucleoside diphosphate kinase homolog 5",
  "gene_symbol": "NME5"
}